{
  "term_label": "chemokine activity",
  "gene": "UniProtKB:Q07325",
  "gene_name": "C-X-C motif chemokine 9",
  "gene_symbol": "CXCL9",
  "term_id": "GO:0008009"
}